{
  "term_label": "Unknown cellular component",
  "gene": "UniProtKB:P0DPQ3",
  "gene_name": "Proline-rich protein 20G",
  "term_id": "UNKNOWN:0003",
  "gene_symbol": "PRR20G"
}